{
  "gene_name": "CCN family member 5",
  "gene": "UniProtKB:O76076",
  "gene_symbol": "CCN5",
  "term_label": "heparin binding",
  "term_id": "GO:0008201"
}